{
  "term_label": "sodium-independent organic anion transport",
  "term_id": "GO:0043252",
  "gene_symbol": "SLCO2B1",
  "gene": "UniProtKB:O94956",
  "gene_name": "Solute carrier organic anion transporter family member 2B1"
}